{
  "gene_name": "WD repeat and FYVE domain-containing protein 1",
  "gene_symbol": "WDFY1",
  "gene": "UniProtKB:Q8IWB7",
  "term_id": "GO:0005769",
  "term_label": "early endosome"
}